{
  "term_id": "GO:0031415",
  "gene_symbol": "NAA16",
  "gene_name": "N-alpha-acetyltransferase 16, NatA auxiliary subunit",
  "term_label": "NatA complex",
  "gene": "UniProtKB:Q6N069"
}